negative regulation of stem cell proliferation [GO:2000647] (biological process) Sources: GOC:dph Relationships: is a type of negative regulation of cell population proliferation [GO:0008285]; is_a regulation of stem cell proliferation [GO:0072091]; negatively regulates stem cell proliferation [GO:0072089] Subtypes: GO:1902034, negative regulation of mesenchymal stem cell proliferation [GO:1902461] Definition: Any process that stops, prevents or reduces the frequency, rate or extent of stem cell proliferation.